{
  "term_id": "UNKNOWN:0001",
  "term_label": "Unknown molecular function",
  "gene": "UniProtKB:A2RUB1",
  "gene_symbol": "MEIOC",
  "gene_name": "Meiosis-specific coiled-coil domain-containing protein MEIOC"
}